{
  "gene_symbol": "EMD",
  "term_label": "nuclear inner membrane",
  "gene_name": "Emerin",
  "term_id": "GO:0005637",
  "gene": "UniProtKB:P50402"
}